{
  "gene": "UniProtKB:Q8WWQ0",
  "gene_name": "PH-interacting protein",
  "term_label": "regulation of cell shape",
  "gene_symbol": "PHIP",
  "term_id": "GO:0008360"
}